{
  "gene_symbol": "PRKD2",
  "gene": "UniProtKB:Q9BZL6",
  "term_id": "GO:0035556",
  "gene_name": "Serine_threonine-protein kinase D2",
  "term_label": "intracellular signal transduction"
}